{
  "term_id": "UNKNOWN:0001",
  "gene": "UniProtKB:Q9H3S7",
  "term_label": "Unknown molecular function",
  "gene_symbol": "PTPN23",
  "gene_name": "Tyrosine-protein phosphatase non-receptor type 23"
}